{
  "gene": "UniProtKB:Q9UBK8",
  "term_id": "GO:0005829",
  "gene_name": "Methionine synthase reductase",
  "term_label": "cytosol",
  "gene_symbol": "MTRR"
}